{
  "term_id": "UNKNOWN:0001",
  "term_label": "Unknown molecular function",
  "gene_symbol": "LINC00303",
  "gene": "UniProtKB:Q3SY05",
  "gene_name": "Putative uncharacterized protein encoded by LINC00303"
}